{
  "gene_symbol": "TMEM174",
  "gene": "UniProtKB:Q8WUU8",
  "gene_name": "Transmembrane protein 174",
  "term_id": "UNKNOWN:0002",
  "term_label": "Unknown biological process"
}